gliotoxin catabolic process [GO:2001309] (biological process) Definition: The chemical reactions and pathways resulting in the breakdown of the epipolythiodioxopiperazine gliotoxin, a poisonous substance produced by some species of fungi. References: PMID:16333108, PMID:17574915, PMID:18272357 Sources: GOC:di Also known as: gliotoxin breakdown, gliotoxin catabolism, gliotoxin degradation Relationships: is_a GO:0043387; is a type of amide metabolic process [GO:0043603]; is a type of GO:0044273; is a type of detoxification of nitrogen compound [GO:0051410]